negative regulation of defense response to insect [GO:1900366] (biological process) Relationships: is a type of negative regulation of response to biotic stimulus [GO:0002832]; is a type of GO:0031348; is a type of negative regulation of response to external stimulus [GO:0032102]; is a type of regulation of defense response to insect [GO:2000068]; negatively regulates GO:0002213 Definition: Any process that stops, prevents or reduces the frequency, rate or extent of defense response to insect. References: PMID:22474183 Sources: GOC:TermGenie Also known as: down regulation of defense response to insect, down regulation of physiological defense response to insect, down-regulation of defense response to insect, down-regulation of physiological defense response to insect, downregulation of defense response to insect, downregulation of physiological defense response to insect, negative regulation of physiological defense response to insect, inhibition of defense response to insect, inhibition of physiological defense response to insect, susceptibility to insect